alpha-beta T cell differentiation involved in immune response [GO:0002293] (biological process) Subtypes: GO:0002294, GO:0002302 Note: Note that immunologists typically use the word 'development' to refer to cells of B or T cell lineages undergoing the process that GO describes as 'cell differentiation'. Relationships: is a type of alpha-beta T cell activation involved in immune response [GO:0002287]; is a type of T cell differentiation involved in immune response [GO:0002292]; is a type of GO:0046632 Definition: The process in which an antigenically naive alpha-beta T cell acquires the specialized features of an effector, regulatory, or memory T cell during an immune response. Effector T cells include cells which provide T cell help or exhibit cytotoxicity towards other cells. Also known as: alpha-beta T cell development involved in immune response, alpha-beta T cell differentiation during immune response, alpha-beta T lymphocyte differentiation during immune response, alpha-beta T-cell differentiation during immune response, alpha-beta T-lymphocyte differentiation during immune response Sources: GOC:add, ISBN:0781735149